{
  "gene": "UniProtKB:Q15797",
  "term_label": "RNA polymerase II cis-regulatory region sequence-specific DNA binding",
  "gene_name": "Mothers against decapentaplegic homolog 1",
  "gene_symbol": "SMAD1",
  "term_id": "GO:0000978"
}